{
  "term_label": "unfolded protein binding",
  "gene_symbol": "CCT5",
  "gene": "UniProtKB:P48643",
  "term_id": "GO:0051082",
  "gene_name": "T-complex protein 1 subunit epsilon"
}